{
  "term_label": "cytosol",
  "gene_symbol": "CDK14",
  "gene_name": "Cyclin-dependent kinase 14",
  "term_id": "GO:0005829",
  "gene": "UniProtKB:O94921"
}